beta-D-fucosidase activity [GO:0033907] (molecular function) Definition: Catalysis of the hydrolysis of terminal non-reducing beta-D-fucose residues in beta-D-fucosides. Sources: EC:3.2.1.38 Also known as: beta-D-fucoside fucohydrolase activity, beta-fucosidase activity Relationships: is a type of GO:0015928